{
  "term_id": "GO:0002376",
  "gene": "UniProtKB:Q14653",
  "term_label": "immune system process",
  "gene_name": "Interferon regulatory factor 3",
  "gene_symbol": "IRF3"
}